{
  "term_id": "GO:0006896",
  "gene_name": "AP-1 complex subunit mu-2",
  "gene_symbol": "AP1M2",
  "term_label": "Golgi to vacuole transport",
  "gene": "UniProtKB:Q9Y6Q5"
}